{
  "term_id": "GO:0031371",
  "gene_symbol": "UBE2V1",
  "gene_name": "Ubiquitin-conjugating enzyme E2 variant 1",
  "term_label": "ubiquitin conjugating enzyme complex",
  "gene": "UniProtKB:Q13404"
}